{
  "term_label": "signal transduction",
  "gene_symbol": "OR1N2",
  "gene_name": "Olfactory receptor 1N2",
  "term_id": "GO:0007165",
  "gene": "UniProtKB:Q8NGR9"
}